alpha4-beta1 integrin-JAM2 complex [GO:0071101] (cellular component) Definition: A protein complex that consists of an alpha4-beta1 integrin complex bound to the cell adhesion molecule JAM2. Also known as: ITGA4-ITGB1-JAM2 complex Relationships: is a type of plasma membrane protein complex [GO:0098797] References: PMID:12070135